{
  "gene_symbol": "STK17A",
  "gene": "UniProtKB:Q9UEE5",
  "term_label": "intracellular signal transduction",
  "term_id": "GO:0035556",
  "gene_name": "Serine_threonine-protein kinase 17A"
}